{
  "term_id": "GO:0016556",
  "gene": "UniProtKB:Q86U44",
  "gene_name": "N6-adenosine-methyltransferase catalytic subunit",
  "gene_symbol": "METTL3",
  "term_label": "mRNA modification"
}